{
  "term_id": "GO:0005525",
  "gene": "UniProtKB:P57735",
  "gene_symbol": "RAB25",
  "gene_name": "Ras-related protein Rab-25",
  "term_label": "GTP binding"
}